{
  "term_id": "GO:0030198",
  "term_label": "extracellular matrix organization",
  "gene_symbol": "COL14A1",
  "gene_name": "Collagen alpha-1(XIV) chain",
  "gene": "UniProtKB:Q05707"
}